female meiotic chromosome movement towards spindle pole [GO:0016345] (biological process) Sources: GOC:ai Definition: The directed movement of chromosomes in the center of the spindle towards the spindle poles, mediated by the shortening of microtubules attached to the chromosomes, during female meiosis. Also known as: female meiotic chromosome movement, chromosome movement towards spindle pole during female meiosis, female meiotic chromosome movement to spindle pole Relationships: is a type of meiotic chromosome movement towards spindle pole [GO:0016344]; is part of female meiosis chromosome segregation [GO:0016321]